{
  "term_label": "nucleus",
  "gene_name": "Tyrosine-protein phosphatase non-receptor type 2",
  "gene": "UniProtKB:P17706",
  "gene_symbol": "PTPN2",
  "term_id": "GO:0005634"
}